{
  "gene": "UniProtKB:Q8IWY8",
  "term_label": "DNA-binding transcription factor activity, RNA polymerase II-specific",
  "term_id": "GO:0000981",
  "gene_name": "Zinc finger and SCAN domain-containing protein 29",
  "gene_symbol": "ZSCAN29"
}